{
  "term_label": "Unknown cellular component",
  "gene_name": "Placenta-specific protein 9",
  "term_id": "UNKNOWN:0003",
  "gene_symbol": "PLAC9",
  "gene": "UniProtKB:Q5JTB6"
}